{
  "gene_name": "Galectin-2",
  "term_id": "UNKNOWN:0003",
  "term_label": "Unknown cellular component",
  "gene_symbol": "LGALS2",
  "gene": "UniProtKB:P05162"
}